negative regulation of semaphorin-plexin signaling pathway [GO:2001261] (biological process) Definition: Any process that stops, prevents or reduces the frequency, rate or extent of semaphorin-plexin signaling pathway. Relationships: is a type of GO:0009968; is a type of regulation of semaphorin-plexin signaling pathway [GO:2001260]; negatively regulates semaphorin-plexin signaling pathway [GO:0071526] Also known as: negative regulation of semaphorin-plexin signalling pathway Sources: GOC:BHF